{
  "term_label": "plasma membrane",
  "term_id": "GO:0005886",
  "gene_name": "Annexin A2",
  "gene": "UniProtKB:P07355",
  "gene_symbol": "ANXA2"
}